alpha-aminoadipate acetyltransferase activity [GO:0043741] (molecular function) Also known as: L-2-aminoadipate N-acetyltransferase activity Definition: Catalysis of the reaction: alpha-aminoadipate + acetyl-CoA = N2-acetyl-alpha-aminoadipate + coenzyme A. Relationships: is_a N-acetyltransferase activity [GO:0008080] References: PMID:10613839, PMID:12925802, PMID:29053735